{
  "gene_symbol": "HOXA10",
  "term_label": "regulation of transcription by RNA polymerase II",
  "term_id": "GO:0006357",
  "gene": "UniProtKB:P31260",
  "gene_name": "Homeobox protein Hox-A10"
}